{
  "term_id": "UNKNOWN:0001",
  "gene_symbol": "PDZD8",
  "term_label": "Unknown molecular function",
  "gene": "UniProtKB:Q8NEN9",
  "gene_name": "PDZ domain-containing protein 8"
}